{
  "gene": "UniProtKB:Q9H4R4",
  "gene_name": "Putative nuclear receptor corepressor 1-like protein NCOR1P1",
  "gene_symbol": "NCOR1P1",
  "term_label": "Unknown cellular component",
  "term_id": "UNKNOWN:0003"
}